{
  "gene_symbol": "IGHV7-81",
  "gene": "UniProtKB:A0A0B4J1V7",
  "term_id": "GO:0003823",
  "term_label": "antigen binding",
  "gene_name": "Probable non-functional immunoglobulin heavy variable 7-81"
}